{
  "gene_symbol": "PPP6R3",
  "term_id": "GO:0005829",
  "gene_name": "Serine_threonine-protein phosphatase 6 regulatory subunit 3",
  "term_label": "cytosol",
  "gene": "UniProtKB:Q5H9R7"
}